{
  "term_label": "aspartic endopeptidase activity, intramembrane cleaving",
  "term_id": "GO:0042500",
  "gene_name": "Presenilin-1",
  "gene_symbol": "PSEN1",
  "gene": "UniProtKB:P49768"
}